{
  "gene": "UniProtKB:Q96M63",
  "gene_name": "Outer dynein arm-docking complex subunit 1",
  "term_label": "cilium movement",
  "gene_symbol": "ODAD1",
  "term_id": "GO:0003341"
}